{
  "term_id": "GO:0005886",
  "gene_symbol": "LNPEP",
  "gene": "UniProtKB:Q9UIQ6",
  "term_label": "plasma membrane",
  "gene_name": "Leucyl-cystinyl aminopeptidase"
}